{
  "gene_symbol": "FRK",
  "gene_name": "Tyrosine-protein kinase FRK",
  "gene": "UniProtKB:P42685",
  "term_id": "GO:0005886",
  "term_label": "plasma membrane"
}